blood vessel morphogenesis [GO:0048514] (biological process) Relationships: is a type of tube morphogenesis [GO:0035239]; is part of blood vessel development [GO:0001568] Subtypes: artery morphogenesis [GO:0048844], venous blood vessel morphogenesis [GO:0048845], GO:0060977, retinal blood vessel morphogenesis [GO:0061304], glomerulus vasculature morphogenesis [GO:0072103] Regulation: negatively regulated by negative regulation of blood vessel morphogenesis [GO:2000181] Definition: The process in which the anatomical structures of blood vessels are generated and organized. The blood vessel is the vasculature carrying blood. Sources: GOC:jid